{
  "gene": "UniProtKB:Q9Y2X9",
  "term_label": "DNA-binding transcription factor activity, RNA polymerase II-specific",
  "term_id": "GO:0000981",
  "gene_name": "Zinc finger protein 281",
  "gene_symbol": "ZNF281"
}